negative regulation of hepatic stellate cell migration [GO:0061871] (biological process) Relationships: is a type of negative regulation of fibroblast migration [GO:0010764]; is a type of regulation of hepatic stellate cell migration [GO:0061869]; negatively regulates GO:0061868 References: PMID:24204762 Definition: Any process that stops, prevents or reduces the frequency, rate or extent of hepatic stellate cell migration.